{
  "gene_symbol": "GABRQ",
  "gene_name": "Gamma-aminobutyric acid receptor subunit theta",
  "term_id": "GO:0005254",
  "term_label": "chloride channel activity",
  "gene": "UniProtKB:Q9UN88"
}